{
  "gene_name": "Transcription initiation factor TFIID subunit 4",
  "term_id": "GO:0016251",
  "gene_symbol": "TAF4",
  "term_label": "RNA polymerase II general transcription initiation factor activity",
  "gene": "UniProtKB:O00268"
}